specification of mesonephric distal tubule identity [GO:0061283] (biological process) Relationships: is a type of specification of mesonephric nephron tubule identity [GO:0061282]; is a type of GO:0072084; is part of mesonephric distal tubule morphogenesis [GO:0061273] Definition: The process in which the distal tubule of the mesonephric nephron acquires its identity. Sources: GOC:mtg_kidney_jan10